{
  "gene_name": "Protein disulfide isomerase CRELD1",
  "term_id": "GO:0005615",
  "term_label": "extracellular space",
  "gene_symbol": "CRELD1",
  "gene": "UniProtKB:Q96HD1"
}